microsporogenesis [GO:0009556] (biological process) Definition: The process in which the microsporocyte undergoes meiosis, giving rise to four haploid microspores. Sources: GOC:mtg_plant, GOC:tb Also known as: microspore development Relationships: is a type of plant-type sporogenesis [GO:0048236]; is part of pollen development [GO:0009555]